{
  "term_label": "Unknown molecular function",
  "term_id": "UNKNOWN:0001",
  "gene_name": "Putative uncharacterized protein FLJ46792",
  "gene_symbol": "Q6ZQY7",
  "gene": "UniProtKB:Q6ZQY7"
}